{
  "term_id": "UNKNOWN:0003",
  "gene_name": "B-cell acute lymphoblastic leukemia-expressed protein",
  "term_label": "Unknown cellular component",
  "gene_symbol": "BLACE",
  "gene": "UniProtKB:A4D250"
}